{
  "term_label": "carnitine metabolic process",
  "gene_name": "Carnitine O-palmitoyltransferase 1, liver isoform",
  "gene_symbol": "CPT1A",
  "gene": "UniProtKB:P50416",
  "term_id": "GO:0009437"
}